caste determination [GO:0048648] (biological process) Subtypes: caste determination, influence by genetic factors [GO:0048649], caste determination, influence by environmental factors [GO:0048650] Sources: GOC:jid Definition: The process in which individuals, having the potential to develop any of several distinct developmental paths, have their individual developmental fate determined in response to environmental and/or genetic cues. Individuals with distinct developmental fates perform different functions in a colony of social insects. Relationships: is a type of GO:0048647